{
  "gene_symbol": "PSMC2",
  "term_label": "proteasome-mediated ubiquitin-dependent protein catabolic process",
  "gene": "UniProtKB:P35998",
  "gene_name": "26S proteasome regulatory subunit 7",
  "term_id": "GO:0043161"
}